gibberellin mediated signaling pathway [GO:0010476] (BP) References: PMID:17521411 Definition: The series of molecular signals generated as a consequence of gibberellin stimulus. Also known as: gibberellin-mediated signalling Subtypes: gibberellic acid mediated signaling pathway [GO:0009740] Relationships: is a type of GO:0009755; BFO_0000050 cellular response to gibberellin stimulus [GO:0071370]